viral capsid, minor subunit [GO:0098018] (cellular component) Relationships: is a type of capsomere [GO:0046727] Also known as: minor capsomere, minor head protein Definition: The part of the viral capsid that comprises the less common capsomere type. For example, in a T=3 icosahedral capsid, which is composed of 12 pentameric and 20 hexameric capsomeres, the pentameric capsomeres are minor subunits. Sources: GOC:bm